negative regulation of myofibroblast contraction [GO:1904329] (biological process) Definition: Any process that stops, prevents or reduces the frequency, rate or extent of myofibroblast contraction. References: PMID:19239477 Sources: GOC:TermGenie, GO_REF:0000058 Relationships: is a type of negative regulation of cellular process [GO:0048523]; is a type of GO:1904328; negatively regulates myofibroblast contraction [GO:1990764] Also known as: down regulation of MF contraction, down regulation of MFB contraction, down regulation of myofibroblast contraction, down-regulation of MF contraction, down-regulation of MFB contraction, down-regulation of myofibroblast contraction, downregulation of MF contraction, downregulation of MFB contraction, downregulation of myofibroblast contraction, negative regulation of MF contraction, negative regulation of MFB contraction, inhibition of MF contraction, inhibition of MFB contraction, inhibition of myofibroblast contraction